{
  "term_label": "NAD+ kinase activity",
  "gene_name": "NAD kinase 2, mitochondrial",
  "term_id": "GO:0003951",
  "gene_symbol": "NADK2",
  "gene": "UniProtKB:Q4G0N4"
}